{
  "term_label": "Unknown cellular component",
  "term_id": "UNKNOWN:0003",
  "gene": "UniProtKB:Q06416",
  "gene_name": "Putative POU domain, class 5, transcription factor 1B",
  "gene_symbol": "POU5F1B"
}